{
  "term_label": "negative regulation of type II interferon production",
  "term_id": "GO:0032689",
  "gene_name": "Galectin-9",
  "gene": "UniProtKB:O00182",
  "gene_symbol": "LGALS9"
}